thienylcyclohexylpiperidine binding [GO:0016596] (molecular function) Sources: GOC:jl Relationships: is a type of sulfur compound binding [GO:1901681] Definition: Binding to thienylcyclohexylpiperidine. Also known as: TCP binding